modulation of excitatory postsynaptic potential [GO:0098815] (biological process) Subtypes: regulation of excitatory postsynaptic membrane potential involved in skeletal muscle contraction [GO:0014853], regulation of mini excitatory postsynaptic potential [GO:0061884], GO:0090394, GO:2000463 Definition: Any process that modulates the frequency, rate or extent of excitatory postsynaptic potential (EPSP). EPSP is a process that leads to a temporary increase in postsynaptic potential due to the flow of positively charged ions into the postsynaptic cell. The flow of ions that causes an EPSP is an excitatory postsynaptic current (EPSC) and makes it easier for the neuron to fire an action potential. Sources: GOC:dos Relationships: is a type of regulation of signal transduction [GO:0009966]; is a type of regulation of nervous system process [GO:0031644]; is a type of regulation of membrane potential [GO:0042391]; is a type of modulation of chemical synaptic transmission [GO:0050804]; regulates GO:0060079